{
  "term_id": "GO:0045334",
  "gene_name": "Phosphatidylinositide phosphatase SAC2",
  "gene_symbol": "INPP5F",
  "gene": "UniProtKB:Q9Y2H2",
  "term_label": "clathrin-coated endocytic vesicle"
}